Cajal body organization [GO:0030576] (biological process) Relationships: is a type of nuclear body organization [GO:0030575] References: PMID:11031238 Sources: GOC:mah Note: See also the cellular component term 'Cajal body ; GO:0015030'. Also known as: Cajal body organisation, Cajal body organization and biogenesis Definition: A process that is carried out at the cellular level which results in the assembly, arrangement of constituent parts, or disassembly of Cajal bodies, nuclear bodies that appear ultrastructurally as a tangle of coiled, electron-dense threads roughly 0.5 micrometers in diameter and are enriched in ribonucleoproteins, and certain general RNA polymerase II transcription factors.